{
  "term_id": "GO:0000977",
  "term_label": "RNA polymerase II transcription regulatory region sequence-specific DNA binding",
  "gene_symbol": "ZBED3",
  "gene_name": "Zinc finger BED domain-containing protein 3",
  "gene": "UniProtKB:Q96IU2"
}